{
  "term_id": "UNKNOWN:0001",
  "term_label": "Unknown molecular function",
  "gene_symbol": "SUMF2",
  "gene": "UniProtKB:Q8NBJ7",
  "gene_name": "Inactive C-alpha-formylglycine-generating enzyme 2"
}